{
  "gene_name": "Collagen alpha-1(XVII) chain",
  "term_id": "GO:0031012",
  "gene_symbol": "COL17A1",
  "term_label": "extracellular matrix",
  "gene": "UniProtKB:Q9UMD9"
}